regulation of UDP-N-acetylglucosamine biosynthetic process [GO:0106278] (biological process) Also known as: regulation of UDP-GlcNAc biosynthetic process, regulation of UDP-N-acetylglucosamine anabolism, regulation of UDP-N-acetylglucosamine biosynthesis, regulation of UDP-N-acetylglucosamine formation, regulation of UDP-N-acetylglucosamine synthesis Subtypes: negative regulation of UDP-N-acetylglucosamine biosynthetic process [GO:0106279], positive regulation of UDP-N-acetylglucosamine biosynthetic process [GO:0106280] References: PMID:32579556 Definition: Any process that modulates the frequency, rate or extent of the UDP-N_acetylglucosamine biosynthetic process. Relationships: is a type of GO:0009889; is a type of regulation of nucleobase-containing compound metabolic process [GO:0019219]; is a type of regulation of phosphorus metabolic process [GO:0051174]; is a type of GO:0062012; regulates UDP-N-acetylglucosamine biosynthetic process [GO:0006048]